semaphorin receptor complex [GO:0002116] (cellular component) References: PMID:10934324, PMID:12367632, PMID:12613544 Sources: GOC:hjd Also known as: plexin-neurophilin complex Definition: A stable binary complex of a semaphorin and a plexin, together forming a functional semaphorin receptor. Relationships: is_a GO:0043235